cellular response to cholesterol [GO:0071397] (biological process) Relationships: is a type of cellular response to sterol [GO:0036315]; is a type of response to cholesterol [GO:0070723]; is_a cellular response to alcohol [GO:0097306] Sources: GOC:mah Definition: Any process that results in a change in state or activity of a cell (in terms of movement, secretion, enzyme production, gene expression, etc.) as a result of a cholesterol stimulus.